{
  "gene_name": "Single-stranded DNA cytosine deaminase",
  "gene": "UniProtKB:Q9GZX7",
  "gene_symbol": "AICDA",
  "term_id": "GO:0045869",
  "term_label": "negative regulation of single stranded viral RNA replication via double stranded DNA intermediate"
}